{
  "gene_symbol": "ZBTB34",
  "gene_name": "Zinc finger and BTB domain-containing protein 34",
  "term_id": "GO:0002682",
  "gene": "UniProtKB:Q8NCN2",
  "term_label": "regulation of immune system process"
}